11beta-hydroxyprogesterone binding [GO:1903879] (molecular function) References: PMID:10802282 Sources: GOC:TermGenie, GOC:mr, GO_REF:0000067 Relationships: is a type of steroid binding [GO:0005496] Definition: Binding to 11beta-hydroxyprogesterone.